{
  "gene_symbol": "INO80E",
  "gene_name": "INO80 complex subunit E",
  "term_id": "UNKNOWN:0001",
  "gene": "UniProtKB:Q8NBZ0",
  "term_label": "Unknown molecular function"
}